{
  "gene_name": "Myb-related protein A",
  "term_label": "mitotic cell cycle",
  "term_id": "GO:0000278",
  "gene": "UniProtKB:P10243",
  "gene_symbol": "MYBL1"
}